{
  "term_id": "GO:0005634",
  "term_label": "nucleus",
  "gene": "UniProtKB:Q9BT49",
  "gene_name": "THAP domain-containing protein 7",
  "gene_symbol": "THAP7"
}